{
  "gene": "UniProtKB:P47211",
  "term_id": "GO:0005886",
  "gene_symbol": "GALR1",
  "term_label": "plasma membrane",
  "gene_name": "Galanin receptor type 1"
}